{
  "term_id": "GO:0000776",
  "gene_symbol": "PLK3",
  "gene_name": "Serine_threonine-protein kinase PLK3",
  "gene": "UniProtKB:Q9H4B4",
  "term_label": "kinetochore"
}